{
  "gene": "UniProtKB:Q8NHC7",
  "gene_symbol": "OR14C36",
  "term_label": "Unknown cellular component",
  "term_id": "UNKNOWN:0003",
  "gene_name": "Olfactory receptor 14C36"
}